{
  "term_id": "GO:0009314",
  "gene_symbol": "POLH",
  "term_label": "response to radiation",
  "gene": "UniProtKB:Q9Y253",
  "gene_name": "DNA polymerase eta"
}